{
  "term_label": "Unknown cellular component",
  "term_id": "UNKNOWN:0003",
  "gene_name": "NXPE family member 4",
  "gene": "UniProtKB:Q6UWF7",
  "gene_symbol": "NXPE4"
}